glucan 1,4-alpha-glucosidase activity [GO:0004339] (molecular function) Definition: Catalysis of the hydrolysis of terminal (1->4)-linked alpha-D-glucose residues successively from non-reducing ends of the chains with release of beta-D-glucose. Sources: EC:3.2.1.3 Also known as: lysosomal alpha-glucosidase activity, glucoamylase activity, 1,4-alpha-D-glucan glucohydrolase activity, amyloglucosidase activity, exo-1,4-alpha-glucosidase activity, gamma-1,4-glucan glucohydrolase activity, gamma-amylase activity, glucose amylase activity Note: Note that this term is not a child of 'alpha-glucosidase activity ; GO:0090599', because in the reaction represented by GO:0004339 results in the release of beta-D-glucose, whereas in GO:0090599 alpha-D-glucose is released. Relationships: is a type of GO:0090599